vasculature development [GO:0001944] (biological process) Definition: The process whose specific outcome is the progression of the vasculature over time, from its formation to the mature structure. The vasculature is an interconnected tubular multi-tissue structure that contains fluid that is actively transported around the organism. Sources: GOC:dph, UBERON:0002409 Also known as: vascular system development Relationships: is a type of system development [GO:0048731]; is part of GO:0072359 Subtypes: lung vasculature development [GO:0060426], GO:0061298, cerebellum vasculature development [GO:0061300], GO:0061437 Regulation: regulated by regulation of vasculature development [GO:1901342]; negatively regulated by GO:1901343; positively regulated by positive regulation of vasculature development [GO:1904018]